L-idonate biosynthetic process [GO:0046182] (biological process) Also known as: L-idonate anabolism, L-idonate biosynthesis, L-idonate formation, L-idonate synthesis Sources: GOC:curators Definition: The chemical reactions and pathways resulting in the formation of L-idonate, the anion of idonic acid, an aldonic acid derived from L-idose, an aldohexose which is epimeric with D-glucose. Relationships: is a type of carbohydrate biosynthetic process [GO:0016051]; is a type of aldonic acid biosynthetic process [GO:0046175]